{
  "gene": "UniProtKB:O14893",
  "gene_name": "Gem-associated protein 2",
  "term_id": "GO:0005634",
  "gene_symbol": "GEMIN2",
  "term_label": "nucleus"
}